pteridine-containing compound catabolic process [GO:0042560] (biological process) Definition: The chemical reactions and pathways resulting in the breakdown of any compound containing pteridine (pyrazino(2,3-dipyrimidine)), e.g. pteroic acid, xanthopterin and folic acid. Sources: GOC:jl, ISBN:0198506732 Also known as: pteridine and derivative catabolic process, pteridine and derivative catabolism, pteridine-containing compound breakdown, pteridine-containing compound catabolism, pteridine-containing compound degradation, pterin catabolic process, pterin catabolism Relationships: is_a catabolic process [GO:0009056]; is a type of pteridine-containing compound metabolic process [GO:0042558] Subtypes: folic acid-containing compound catabolic process [GO:0009397], pteridine catabolic process [GO:0019990], GO:0046147, GO:1901284, 5,6,7,8-tetrahydrosarcinapterin catabolic process [GO:1901854]